{
  "gene_symbol": "CDH2",
  "gene_name": "Cadherin-2",
  "term_id": "GO:0016477",
  "term_label": "cell migration",
  "gene": "UniProtKB:P19022"
}